{
  "term_label": "plasma membrane",
  "gene_symbol": "LPAR4",
  "gene_name": "Lysophosphatidic acid receptor 4",
  "term_id": "GO:0005886",
  "gene": "UniProtKB:Q99677"
}